{
  "gene_name": "Muscleblind-like protein 2",
  "term_label": "cytoplasm",
  "gene": "UniProtKB:Q5VZF2",
  "term_id": "GO:0005737",
  "gene_symbol": "MBNL2"
}